{
  "term_label": "DNA-directed RNA polymerase activity",
  "term_id": "GO:0003899",
  "gene": "UniProtKB:O15160",
  "gene_name": "DNA-directed RNA polymerases I and III subunit RPAC1",
  "gene_symbol": "POLR1C"
}